glycerol-3-phosphate transmembrane transport [GO:0015794] (biological process) Definition: The process in which glycerol-3-phosphate is transported across a membrane. Glycerol-3-phosphate is a phosphoric monoester of glycerol. Relationships: is_a organic anion transport [GO:0015711]; is a type of organophosphate ester transport [GO:0015748]; is a type of transmembrane transport [GO:0055085]; is a type of carbohydrate derivative transport [GO:1901264] Also known as: glycerol-3-phosphate transport Sources: GOC:ai